{
  "gene_name": "Upstream-binding factor 1-like protein 1",
  "term_label": "RNA polymerase I general transcription initiation factor activity",
  "term_id": "GO:0001181",
  "gene_symbol": "UBTFL1",
  "gene": "UniProtKB:P0CB47"
}